{
  "gene_symbol": "PSAT1",
  "gene_name": "Phosphoserine aminotransferase",
  "term_label": "cytoplasm",
  "term_id": "GO:0005737",
  "gene": "UniProtKB:Q9Y617"
}